{
  "term_id": "GO:0006302",
  "gene_name": "Putative histone PARylation factor 1-like",
  "term_label": "double-strand break repair",
  "gene": "UniProtKB:A8MVJ9",
  "gene_symbol": "A8MVJ9"
}